mitochondrial small ribosomal subunit binding [GO:0180065] (molecular function) Definition: Binding to a mitochondrial small ribosomal subunit. Also known as: mtSSU binding Relationships: is_a GO:0097177 References: PMID:40427588